positive regulation of transmembrane receptor protein serine/threonine kinase signaling pathway [GO:0090100] (biological process) Definition: Any process that increases the rate, frequency, or extent of the series of molecular signals generated as a consequence of a transmembrane receptor serine/threonine kinase binding to its physiological ligand. Also known as: positive regulation of transmembrane receptor protein serine/threonine kinase signalling pathway Sources: GOC:dph, GOC:tb Relationships: is a type of GO:0009967; is a type of regulation of transmembrane receptor protein serine/threonine kinase signaling pathway [GO:0090092]; positively regulates GO:0007178 Subtypes: positive regulation of transforming growth factor beta receptor signaling pathway [GO:0030511], positive regulation of BMP signaling pathway [GO:0030513], positive regulation of activin receptor signaling pathway [GO:0032927], positive regulation of SMAD protein signal transduction [GO:0060391], positive regulation of anti-Mullerian hormone signaling pathway [GO:1902614]